{
  "term_id": "GO:0005096",
  "gene_symbol": "ASAP1",
  "gene_name": "Arf-GAP with SH3 domain, ANK repeat and PH domain-containing protein 1",
  "term_label": "GTPase activator activity",
  "gene": "UniProtKB:Q9ULH1"
}